{
  "gene_symbol": "SH3RF2",
  "term_label": "negative regulation of apoptotic process",
  "gene": "UniProtKB:Q8TEC5",
  "gene_name": "E3 ubiquitin-protein ligase SH3RF2",
  "term_id": "GO:0043066"
}